{
  "gene": "UniProtKB:P28324",
  "term_id": "GO:0030154",
  "gene_symbol": "ELK4",
  "gene_name": "ETS domain-containing protein Elk-4",
  "term_label": "cell differentiation"
}